{
  "gene": "UniProtKB:Q49A26",
  "gene_symbol": "GLYR1",
  "gene_name": "Cytokine-like nuclear factor N-PAC",
  "term_id": "GO:0140673",
  "term_label": "transcription elongation-coupled chromatin remodeling"
}